induction of conjugation upon nutrient starvation [GO:0031140] (biological process) Relationships: is a type of induction of conjugation with cellular fusion [GO:0010514] Sources: GOC:mah Subtypes: induction of conjugation upon carbon starvation [GO:0031141], induction of conjugation upon nitrogen starvation [GO:0031142] Definition: The process in which a cell initiates conjugation with cellular fusion upon starvation for one or more nutrients.